{
  "term_label": "RecQ family helicase-topoisomerase III complex",
  "term_id": "GO:0031422",
  "gene": "UniProtKB:Q9H9A7",
  "gene_symbol": "RMI1",
  "gene_name": "RecQ-mediated genome instability protein 1"
}